transforming growth factor beta receptor signaling pathway [GO:0007179] (biological process) Relationships: is a type of transforming growth factor beta receptor superfamily signaling pathway [GO:0141091]; is part of cellular response to transforming growth factor beta stimulus [GO:0071560] Sources: GOC:BHF, GOC:mah, GOC:signaling Regulation: regulated by regulation of transforming growth factor beta receptor signaling pathway [GO:0017015]; positively regulated by GO:0030511; RO_0002212 by negative regulation of transforming growth factor beta receptor signaling pathway [GO:0030512] Definition: The series of molecular signals initiated by an extracellular ligand binding to a transforming growth factor beta receptor on the surface of a target cell, and ending with the regulation of a downstream cellular process, e.g. transcription. Also known as: TGF-beta receptor signaling pathway, TGF-beta receptor signalling pathway, TGFbeta receptor signaling pathway, TGFbeta receptor signalling pathway, transforming growth factor beta receptor signalling pathway